{
  "gene_symbol": "BORA",
  "term_label": "regulation of mitotic spindle organization",
  "term_id": "GO:0060236",
  "gene": "UniProtKB:Q6PGQ7",
  "gene_name": "Protein aurora borealis"
}